{
  "term_label": "Unknown cellular component",
  "gene_name": "Protein FAM236A",
  "gene_symbol": "FAM236A",
  "term_id": "UNKNOWN:0003",
  "gene": "UniProtKB:A0A1B0GUQ0"
}